{
  "term_label": "adenylate cyclase-activating G protein-coupled receptor signaling pathway",
  "gene": "UniProtKB:Q8IZF5",
  "gene_name": "Adhesion G-protein coupled receptor F3",
  "gene_symbol": "ADGRF3",
  "term_id": "GO:0007189"
}